{
  "term_id": "GO:0007271",
  "gene": "UniProtKB:Q7Z5B4",
  "gene_symbol": "RIC3",
  "term_label": "synaptic transmission, cholinergic",
  "gene_name": "Protein RIC-3"
}